nuclear pore central transport channel [GO:0044613] (cellular component) Definition: The central substructure of the nuclear pore complex (NPC), through which nucleocytoplasmic transport of RNAs, proteins and small molecules occurs. The central transport channel is filled with FG-nucleoporins, which form a selective barrier and provide a series of binding sites for transporter proteins. Characterized S. cerevisiae FG-nucleoporins include Nup159p, Nup145Np, Nup116p, Nup100p, Nsp1p, Nup57p, Nup49p, Nup42p, Nup53p, Nup59p/Asm4p, Nup60p and Nup1. Characterized vertebrate FG-nucleoporins include Nup214, Nup98, Nup62, Nup54, Nup58/45, NLP1, and Nup153. Relationships: is a type of GO:0140513; BFO_0000050 nuclear pore [GO:0005643] References: PMID:18046406, PMID:19524430, PMID:20947011, PMID:22419078 Sources: GOC:dgf Also known as: nuclear pore central channel, nuclear pore central plug, nuclear pore transport channel, karyopherin docking complex